DNA endoreduplication [GO:0042023] (biological process) Relationships: is a type of GO:0044786; has part DNA replication initiation [GO:0006270] Regulation: regulated by regulation of DNA endoreduplication [GO:0032875]; negatively regulated by negative regulation of DNA endoreduplication [GO:0032876]; positively regulated by positive regulation of DNA endoreduplication [GO:0032877] Note: Note that this term is only to be used in situations were this process occurs normally. Not to be used to describe mutant or diseased states. Sources: GOC:jl, GOC:vw Also known as: DNA endoreplication, DNA re-duplication Definition: Regulated re-replication of DNA within a single cell cycle, resulting in an increased cell ploidy. An example of this process occurs in the synthesis of Drosophila salivary gland cell polytene chromosomes.